regulation of protein stability [GO:0031647] (biological process) Relationships: is_a GO:0065008 Subtypes: protein destabilization [GO:0031648], maintenance of unfolded protein [GO:0036506], protein stabilization [GO:0050821] Definition: Any process that affects the structure and integrity of a protein, altering the likelihood of its degradation or aggregation. Sources: GOC:dph, GOC:mah, GOC:tb